NADP+ metabolic process [GO:0006739] (biological process) Regulation: regulated by regulation of NADP metabolic process [GO:1902031] Subtypes: NADPH regeneration [GO:0006740], NADP+ biosynthetic process [GO:0006741], NADP+ catabolic process [GO:0006742] Sources: GOC:mah Relationships: is a type of GO:0006163; is a type of nicotinamide nucleotide metabolic process [GO:0046496] Definition: The chemical reactions and pathways involving nicotinamide adenine dinucleotide phosphate (NADP+), a coenzyme that interconverts with its reduced form, NADPH, in many redox and biosynthetic reactions. Also known as: NADP (oxidized) metabolic process, NADP (oxidized) metabolism, NADP (reduced) metabolic process, NADP (reduced) metabolism, NADP metabolic process, NADP metabolism, NADPH metabolic process, NADPH metabolism, nicotinamide adenine dinucleotide phosphate metabolic process, nicotinamide adenine dinucleotide phosphate metabolism, oxidized NADP metabolic process, oxidized NADP metabolism, oxidized nicotinamide adenine dinucleotide phosphate metabolic process, oxidized nicotinamide adenine dinucleotide phosphate metabolism, reduced NADP metabolic process, reduced NADP metabolism, reduced nicotinamide adenine dinucleotide phosphate metabolic process, reduced nicotinamide adenine dinucleotide phosphate metabolism, NAD phosphorylation and dephosphorylation